negative regulation of pseudohyphal growth [GO:2000221] (biological process) Definition: Any process that stops, prevents, or reduces the frequency, rate or extent of pseudohyphal growth. Sources: GOC:mah Relationships: is a type of GO:0030308; is a type of GO:0070785; is a type of GO:2000220; negatively regulates GO:0007124